{
  "term_id": "GO:0016477",
  "gene_symbol": "RNH1",
  "gene": "UniProtKB:P13489",
  "gene_name": "Ribonuclease inhibitor",
  "term_label": "cell migration"
}